{
  "gene_symbol": "ATP2C1",
  "gene_name": "Calcium-transporting ATPase type 2C member 1",
  "term_id": "GO:0070588",
  "term_label": "calcium ion transmembrane transport",
  "gene": "UniProtKB:P98194"
}